lactose transport [GO:0015767] (biological process) Sources: GOC:ai Definition: The directed movement of lactose into, out of or within a cell, or between cells, by means of some agent such as a transporter or pore. Lactose is a disaccharide 4-O-beta-D-galactopyranosyl-D-glucose, and constitutes roughly 5% of the milk in almost all mammals. Relationships: is a type of disaccharide transport [GO:0015766]